{
  "term_id": "GO:0008017",
  "gene_symbol": "DNM3",
  "term_label": "microtubule binding",
  "gene_name": "Dynamin-3",
  "gene": "UniProtKB:Q9UQ16"
}